{
  "gene": "UniProtKB:Q86SG6",
  "gene_name": "Serine_threonine-protein kinase Nek8",
  "term_label": "heart development",
  "gene_symbol": "NEK8",
  "term_id": "GO:0007507"
}